{
  "gene_symbol": "FTMT",
  "term_label": "Unknown biological process",
  "term_id": "UNKNOWN:0002",
  "gene": "UniProtKB:Q8N4E7",
  "gene_name": "Ferritin, mitochondrial"
}